{
  "term_id": "GO:0005254",
  "term_label": "chloride channel activity",
  "gene": "UniProtKB:Q96S66",
  "gene_symbol": "CLCC1",
  "gene_name": "Chloride channel CLIC-like protein 1"
}